{
  "gene_name": "Protein FAM104A",
  "term_label": "Unknown cellular component",
  "term_id": "UNKNOWN:0003",
  "gene_symbol": "FAM104A",
  "gene": "UniProtKB:Q969W3"
}